RNA-DNA hybrid ribonuclease activity [GO:0004523] (molecular function) Relationships: is a type of RNA endonuclease activity producing 5'-phosphomonoesters, hydrolytic mechanism [GO:0016891] Note: Note that the EC recommended name for this enzyme activity is 'calf thymus ribonuclease H', even though it is found in many species. Sources: EC:3.1.26.4 Also known as: RNase H activity, calf thymus ribonuclease H activity, ribonuclease H activity, RNase H1 activity, RNase H2 activity, RNase H3 activity, endoribonuclease0 H activity, ribonuclease H1 activity, ribonuclease H2 activity, ribonuclease H3 activity, RNA*DNA hybrid ribonucleotidohydrolase activity, endoribonuclease H, endoribonuclease H (calf thymus), hybrid nuclease activity, hybrid ribonuclease activity, hybridase (ribonuclease H), hybridase activity Definition: Catalysis of the endonucleolytic cleavage of RNA in RNA-DNA hybrids to 5'-phosphomonoesters.